protein arginine phosphatase activity [GO:0098627] (molecular function) Definition: Catalysis of the reaction: phospho-L-arginyl-[protein] +H2O = L-arginyl-[protein] + phosphate. Relationships: is a type of phosphoprotein phosphatase activity [GO:0004721]; is a type of GO:0016825 References: PMID:23770242 Sources: RHEA:43380